positive regulation of muscle hypertrophy [GO:0014742] (biological process) Definition: Any process that activates or increases the frequency, rate or extent of muscle hypertrophy. Sources: GOC:mtg_muscle Relationships: is a type of regulation of muscle hypertrophy [GO:0014743]; is a type of positive regulation of multicellular organismal process [GO:0051240]; positively regulates GO:0014896 Subtypes: positive regulation of cardiac muscle hypertrophy [GO:0010613], positive regulation of skeletal muscle hypertrophy [GO:1904206], positive regulation of smooth muscle hypertrophy [GO:1905149]